{
  "term_label": "regulation of translational termination",
  "term_id": "GO:0006449",
  "gene": "UniProtKB:Q8N543",
  "gene_name": "Prolyl 3-hydroxylase OGFOD1",
  "gene_symbol": "OGFOD1"
}